manchette assembly [GO:1905198] (BP) Definition: The aggregation, arrangement and bonding together of a set of components to form a manchette. References: PMID:22319670, PMID:24440897, PMID:26792866 Sources: GOC:TermGenie, GOC:krc, GO_REF:0000079 Also known as: manchette formation Relationships: is a type of cellular component assembly [GO:0022607]; is part of spermatid development [GO:0007286]